{
  "term_label": "positive regulation of ERK1 and ERK2 cascade",
  "gene": "UniProtKB:Q9NRA1",
  "term_id": "GO:0070374",
  "gene_name": "Platelet-derived growth factor C",
  "gene_symbol": "PDGFC"
}